{
  "gene": "UniProtKB:Q9P2J3",
  "term_label": "proteasome-mediated ubiquitin-dependent protein catabolic process",
  "gene_symbol": "KLHL9",
  "term_id": "GO:0043161",
  "gene_name": "Kelch-like protein 9"
}